tube formation [GO:0035148] (biological process) Sources: GOC:bf Relationships: is a type of GO:0048646; is part of tube morphogenesis [GO:0035239] Subtypes: lumen formation, open tracheal system [GO:0035149], GO:0060605, GO:0060606, GO:0060876, epithelial tube formation [GO:0072175] Also known as: tube lumen formation, lumen formation in an anatomical structure Definition: Creation of the central hole of a tube in an anatomical structure through which gases and/or liquids flow.